mesonephric mesenchymal cell proliferation involved in mesonephros development [GO:0061222] (biological process) Sources: GOC:mtg_kidney_jan10 Definition: The multiplication or reproduction of cells, resulting in the expansion of a mesonephric mesenchymal cell population. Relationships: is a type of cell proliferation involved in mesonephros development [GO:0061209]; is a type of GO:0072135; is part of GO:0061219